{
  "gene_symbol": "LCN1",
  "gene": "UniProtKB:P31025",
  "term_id": "UNKNOWN:0001",
  "gene_name": "Lipocalin-1",
  "term_label": "Unknown molecular function"
}